granulocyte colony-stimulating factor signaling pathway [GO:0038158] (biological process) Sources: GOC:nhn, GOC:signaling Relationships: is a type of cytokine-mediated signaling pathway [GO:0019221] Also known as: CSF3 signaling pathway, G-CSF receptor signaling pathway, G-CSF signaling pathway, granulocyte colony-stimulating factor receptor signaling pathway, granulocyte colony-stimulating factor signalling pathway Definition: The series of molecular signals initiated by the binding of the cytokine granulocyte colony-stimulating factor (G-CSF) to its receptor on the surface of a target cell, and ending with the regulation of a downstream cellular process, e.g. transcription. G-CSF binds to the receptor (CSF3R).